{
  "term_id": "GO:0005634",
  "term_label": "nucleus",
  "gene_name": "Ubiquitin carboxyl-terminal hydrolase 34",
  "gene_symbol": "USP34",
  "gene": "UniProtKB:Q70CQ2"
}